{
  "gene": "UniProtKB:Q8NGN8",
  "term_id": "GO:0005886",
  "gene_name": "Putative olfactory receptor 4A4",
  "gene_symbol": "OR4A4P",
  "term_label": "plasma membrane"
}